{
  "gene": "UniProtKB:Q01780",
  "term_label": "single-stranded RNA binding",
  "gene_name": "Exosome component 10",
  "gene_symbol": "EXOSC10",
  "term_id": "GO:0003727"
}